{
  "gene_symbol": "VTN",
  "term_id": "GO:0005615",
  "gene": "UniProtKB:P04004",
  "gene_name": "Vitronectin",
  "term_label": "extracellular space"
}